{
  "term_label": "cytoplasm",
  "gene": "UniProtKB:Q9NV79",
  "gene_symbol": "PCMTD2",
  "term_id": "GO:0005737",
  "gene_name": "Protein-L-isoaspartate O-methyltransferase domain-containing protein 2"
}